{
  "gene": "UniProtKB:P49019",
  "term_label": "nicotinic acid receptor activity",
  "term_id": "GO:0070553",
  "gene_symbol": "HCAR3",
  "gene_name": "Hydroxycarboxylic acid receptor 3"
}